peptidyl-tryptophan modification [GO:0018211] (biological process) Relationships: is a type of peptidyl-amino acid modification [GO:0018193] Sources: GOC:isa_complete Definition: The chemical alteration of a tryptophan residue in a peptide.